{
  "term_id": "GO:0005549",
  "gene_symbol": "OR6N2",
  "gene": "UniProtKB:Q8NGY6",
  "term_label": "odorant binding",
  "gene_name": "Olfactory receptor 6N2"
}